{
  "gene_symbol": "VTA1",
  "gene": "UniProtKB:Q9NP79",
  "gene_name": "Vacuolar protein sorting-associated protein VTA1 homolog",
  "term_id": "UNKNOWN:0001",
  "term_label": "Unknown molecular function"
}